{
  "term_label": "cysteine-type deubiquitinase activity",
  "term_id": "GO:0004843",
  "gene": "UniProtKB:P0C7H9",
  "gene_name": "Inactive ubiquitin carboxyl-terminal hydrolase 17-like protein 7",
  "gene_symbol": "USP17L7"
}